primary adaptive immune response involving T cells and B cells [GO:0090721] (biological process) Definition: An adaptive immune response mediated by naive T or B cells against an antigen not previously encountered by immune system. Relationships: is_a adaptive immune response based on somatic recombination of immune receptors built from immunoglobulin superfamily domains [GO:0002460]; is a type of GO:0090720 References: PMID:26831526 Sources: GOC:add